{
  "term_id": "GO:0000281",
  "term_label": "mitotic cytokinesis",
  "gene_name": "Nucleolar and spindle-associated protein 1",
  "gene_symbol": "NUSAP1",
  "gene": "UniProtKB:Q9BXS6"
}